guanylyltransferase activity [GO:0070568] (molecular function) Definition: Catalysis of the transfer of a guanylyl group to an acceptor. Sources: GOC:mah Relationships: is a type of nucleotidyltransferase activity [GO:0016779] Subtypes: mannose-1-phosphate guanylyltransferase (GTP) activity [GO:0004475], RNA guanylyltransferase activity [GO:0008192], GO:0008820, GO:0008928, GDP-galactose:mannose-1-phosphate guanylyltransferase activity [GO:0010471], GO:0010472, GO:0010473, phospholactate guanylyltransferase activity [GO:0043814], GO:0044600, fucose-1-phosphate guanylyltransferase activity [GO:0047341], glucose-1-phosphate guanylyltransferase activity [GO:0047344], GTP guanylyltransferase activity [GO:0047351], GTP:coenzyme F420 guanyltransferase activity [GO:0052754], GO:0061603, GDP-L-galactose phosphorylase activity [GO:0080047], GDP-D-glucose phosphorylase activity [GO:0080048], pyridinol guanylyltransferase activity [GO:0160298]